{
  "gene_name": "Neuronal acetylcholine receptor subunit alpha-5",
  "gene_symbol": "CHRNA5",
  "term_label": "acetylcholine-gated monoatomic cation-selective channel activity",
  "term_id": "GO:0022848",
  "gene": "UniProtKB:P30532"
}